Z chromosome [GO:0000807] (CC) Definition: The sex chromosome present in both sexes of species in which the female is the heterogametic sex. Two copies of the Z chromosome are present in each somatic cell of males and one copy is present in females. References: PMID:20622855 Sources: GOC:mah, GOC:mr, ISBN:0321000382 Relationships: is a type of GO:0000803